{
  "term_id": "GO:0015824",
  "term_label": "proline transport",
  "gene_name": "Sodium-dependent neutral amino acid transporter SLC6A17",
  "gene_symbol": "SLC6A17",
  "gene": "UniProtKB:Q9H1V8"
}